{
  "gene": "UniProtKB:Q9Y2X3",
  "term_label": "box C/D methylation guide snoRNP complex",
  "term_id": "GO:0031428",
  "gene_name": "Nucleolar protein 58",
  "gene_symbol": "NOP58"
}